{
  "term_label": "DNA-binding transcription factor activity, RNA polymerase II-specific",
  "term_id": "GO:0000981",
  "gene": "UniProtKB:Q9H175",
  "gene_name": "Cysteine_serine-rich nuclear protein 2",
  "gene_symbol": "CSRNP2"
}